{
  "gene_name": "Ribonuclease 7",
  "gene": "UniProtKB:Q9H1E1",
  "gene_symbol": "RNASE7",
  "term_id": "GO:0045087",
  "term_label": "innate immune response"
}